RNA dinucleotide insertion [GO:0070707] (BP) Sources: GOC:cb, GOC:mah Subtypes: RNA adenosine-uridine insertion [GO:0070711], GO:0070712, RNA guanosine-cytidine insertion [GO:0070713], GO:0070714 Relationships: is a type of RNA nucleotide insertion [GO:0070705] Definition: The modification of an RNA molecule by insertion of a dinucleotide.